reticuline oxidase activity [GO:0050468] (molecular function) Relationships: is a type of GO:0046993 Sources: RHEA:19885 Definition: Catalysis of the reaction: (S)-reticuline + O2 = (S)-scoulerine + H2O2 + H+. Also acts on related compounds, converting the N-methyl group into the methylene bridge ('berberine bridge') of (S)- tetrahydroprotoberberines. Also known as: (S)-reticuline:oxygen oxidoreductase (methylene-bridge-forming), BBE, berberine bridge enzyme activity, berberine-bridge-forming enzyme activity, tetrahydroprotoberberine synthase activity